{
  "gene": "UniProtKB:O75344",
  "term_label": "spermatogenesis",
  "gene_symbol": "FKBP6",
  "gene_name": "Inactive peptidyl-prolyl cis-trans isomerase FKBP6",
  "term_id": "GO:0007283"
}